{
  "term_id": "GO:0005576",
  "gene": "UniProtKB:Q8NBI3",
  "gene_symbol": "DRAXIN",
  "gene_name": "Draxin",
  "term_label": "extracellular region"
}